{
  "term_id": "UNKNOWN:0003",
  "gene_name": "Late cornified envelope protein 1F",
  "term_label": "Unknown cellular component",
  "gene": "UniProtKB:Q5T754",
  "gene_symbol": "LCE1F"
}